clathrin adaptor complex [GO:0030131] (CC) Sources: GOC:mah Definition: A membrane coat adaptor complex that links clathrin to a membrane. Relationships: is a type of AP-type membrane coat adaptor complex [GO:0030119]; is part of clathrin coat [GO:0030118] Subtypes: AP-1 adaptor complex [GO:0030121], AP-2 adaptor complex [GO:0030122]